{
  "term_id": "GO:0006357",
  "gene_symbol": "TFDP3",
  "gene": "UniProtKB:Q5H9I0",
  "term_label": "regulation of transcription by RNA polymerase II",
  "gene_name": "Transcription factor Dp family member 3"
}